CD8-positive, alpha-beta T cell lineage commitment [GO:0043375] (biological process) Sources: ISBN:0781735149 Definition: The process in which an immature T cell becomes committed to becoming a CD8-positive, alpha-beta T cell. Also known as: CD8-positive, alpha-beta T cell fate commitment, CD8-positive, alpha-beta T lymphocyte lineage commitment, CD8-positive, alpha-beta T-cell lineage commitment, CD8-positive, alpha-beta T-lymphocyte lineage commitment Relationships: is a type of alpha-beta T cell lineage commitment [GO:0002363]; is a type of CD4-positive or CD8-positive, alpha-beta T cell lineage commitment [GO:0043369]; is part of CD8-positive, alpha-beta T cell differentiation [GO:0043374]